{
  "gene_name": "Olfactory receptor 6P1",
  "gene": "UniProtKB:Q8NGX9",
  "term_id": "GO:0005886",
  "gene_symbol": "OR6P1",
  "term_label": "plasma membrane"
}